{
  "gene_name": "Isocitrate dehydrogenase [NAD] subunit gamma, mitochondrial",
  "term_label": "tricarboxylic acid cycle",
  "term_id": "GO:0006099",
  "gene": "UniProtKB:P51553",
  "gene_symbol": "IDH3G"
}